{
  "gene_name": "Calcyclin-binding protein",
  "term_id": "GO:0005634",
  "gene_symbol": "CACYBP",
  "term_label": "nucleus",
  "gene": "UniProtKB:Q9HB71"
}